floor plate development [GO:0033504] (biological process) Sources: GOC:dh Definition: The progression of the floor plate over time from its initial formation until its mature state. Relationships: is a type of anatomical structure development [GO:0048856]; is part of neural tube development [GO:0021915]